{
  "term_label": "Unknown molecular function",
  "gene_name": "Reticulophagy regulator 1",
  "term_id": "UNKNOWN:0001",
  "gene": "UniProtKB:Q9H6L5",
  "gene_symbol": "RETREG1"
}